mucin granule [GO:0098594] (cellular component) References: PMID:16377632 Relationships: is a type of secretory granule [GO:0030141] Definition: A secretory granule that contains mucin.